specification of pronephric distal tubule identity [GO:0039010] (biological process) Sources: GOC:mtg_kidney_jan10 Definition: The process in which the distal tubule of the pronephric nephron acquires its identity. Relationships: is a type of specification of pronephric tubule identity [GO:0039005]; is a type of GO:0072084; is a type of proximal/distal pattern formation involved in pronephric nephron development [GO:0072196]; is part of pronephric distal tubule morphogenesis [GO:0039013]